dentin extracellular matrix secretion [GO:0070468] (biological process) Definition: The regulated release by odontoblasts of the extracellular matrix constituents, including collagen, that form the basis of dentin. Also known as: dentin secretion, dentine secretion, predentin secretion Relationships: is a type of extracellular matrix constituent secretion [GO:0070278]; is part of GO:0042475 References: PMID:12856968 Sources: GOC:mah